{
  "gene_symbol": "VAX2",
  "gene": "UniProtKB:Q9UIW0",
  "term_label": "regulation of transcription by RNA polymerase II",
  "term_id": "GO:0006357",
  "gene_name": "Ventral anterior homeobox 2"
}